{
  "term_label": "interleukin-10-mediated signaling pathway",
  "term_id": "GO:0140105",
  "gene_symbol": "LILRA1",
  "gene": "UniProtKB:O75019",
  "gene_name": "Leukocyte immunoglobulin-like receptor subfamily A member 1"
}